{
  "gene_name": "Putative protocadherin beta-18",
  "gene_symbol": "PCDHB18P",
  "term_label": "cell adhesion",
  "term_id": "GO:0007155",
  "gene": "UniProtKB:Q96TA0"
}